{
  "term_label": "nucleus",
  "term_id": "GO:0005634",
  "gene": "UniProtKB:P0DP25",
  "gene_name": "Calmodulin-3",
  "gene_symbol": "CALM3"
}